{
  "term_label": "Unknown cellular component",
  "gene_name": "Protein GREB1",
  "term_id": "UNKNOWN:0003",
  "gene_symbol": "GREB1",
  "gene": "UniProtKB:Q4ZG55"
}